{
  "term_id": "GO:0005634",
  "gene_name": "Proteasome assembly chaperone 2",
  "gene_symbol": "PSMG2",
  "gene": "UniProtKB:Q969U7",
  "term_label": "nucleus"
}